{
  "term_id": "UNKNOWN:0001",
  "term_label": "Unknown molecular function",
  "gene_symbol": "CC2D2A",
  "gene": "UniProtKB:Q9P2K1",
  "gene_name": "Coiled-coil and C2 domain-containing protein 2A"
}